{
  "term_label": "Unknown molecular function",
  "gene": "UniProtKB:Q8IXS0",
  "gene_name": "Protein FAM217A",
  "gene_symbol": "FAM217A",
  "term_id": "UNKNOWN:0001"
}